tetrasaccharide transport [GO:2001098] (biological process) Definition: The directed movement of a tetrasaccharideacetate into, out of or within a cell, or between cells, by means of some agent such as a transporter or pore. Relationships: is a type of oligosaccharide transport [GO:0015772] Subtypes: maltotetraose transport [GO:2001099] Sources: GOC:mengo_curators